{
  "gene": "UniProtKB:Q8WVF1",
  "gene_symbol": "OSCP1",
  "gene_name": "Protein OSCP1",
  "term_id": "UNKNOWN:0001",
  "term_label": "Unknown molecular function"
}